{
  "gene": "UniProtKB:P30038",
  "gene_name": "Delta-1-pyrroline-5-carboxylate dehydrogenase, mitochondrial",
  "term_label": "L-glutamate gamma-semialdehyde dehydrogenase activity",
  "gene_symbol": "ALDH4A1",
  "term_id": "GO:0003842"
}